teichoic acid catabolic process [GO:0070393] (biological process) Subtypes: GO:0070396, wall teichoic acid catabolic process [GO:0070399] Definition: The chemical reactions and pathways resulting in the breakdown of teichoic acid, which is a major component of the cell wall of Gram-positive bacteria and typically consists of a polymer of glycerol-phosphate or ribitol-phosphate to which are attached glycosyl and D-alanyl ester residues. Relationships: is a type of macromolecule catabolic process [GO:0009057]; is a type of teichoic acid metabolic process [GO:0046374]; is a type of carbohydrate derivative catabolic process [GO:1901136] Also known as: teichoic acid breakdown, teichoic acid catabolism, teichoic acid degradation References: PMID:14665680 Sources: GOC:add